{
  "term_label": "anatomical structure morphogenesis",
  "gene_symbol": "FOXL1",
  "term_id": "GO:0009653",
  "gene_name": "Forkhead box protein L1",
  "gene": "UniProtKB:Q12952"
}